arachidonate 8,9-epoxygenase activity [GO:0106302] (molecular function) Also known as: arachidonic acid 8,9-epoxygenase activity References: PMID:10491410, PMID:8246128 Sources: RHEA:64984 Relationships: is a type of arachidonate epoxygenase activity [GO:0008392] Definition: Catalysis of an NADPH- and oxygen-dependent reaction that converts arachidonic acid to cis-8,9-epoxyeicosatrienoic acid.